random inactivation of X chromosome [GO:0060816] (biological process) Also known as: rXCI Definition: Compensating for the two-fold variation in X-chromosome:autosome ratios between sexes by a global inactivation of all, or most of, the genes on either the paternal or maternal X-chromosome in the XX sex. Relationships: is_a dosage compensation by inactivation of X chromosome [GO:0009048] References: PMID:32189388 Sources: GOC:dph, GOC:sdb_2009, GOC:tb